{
  "gene_symbol": "INS",
  "gene": "UniProtKB:P01308",
  "term_label": "hormone activity",
  "term_id": "GO:0005179",
  "gene_name": "Insulin"
}